{
  "term_id": "GO:0005634",
  "gene": "UniProtKB:Q9Y4A8",
  "gene_name": "Nuclear factor erythroid 2-related factor 3",
  "gene_symbol": "NFE2L3",
  "term_label": "nucleus"
}